protein biosynthetic process [GO:0160307] (biological process) Also known as: protein biosynthesis, protein synthesis Relationships: is_a macromolecule biosynthetic process [GO:0009059]; is a type of protein metabolic process [GO:0019538]; is part of GO:0010467; has part tRNA aminoacylation [GO:0043039] Definition: The chemical reactions and pathways resulting in the formation of protein. Sources: Wikipedia:Protein_biosynthesis